Ras protein signal transduction [GO:0007265] (biological process) Also known as: Ras mediated signal transduction Regulation: RO_0002211 by regulation of Ras protein signal transduction [GO:0046578]; positively regulated by GO:0046579; negatively regulated by negative regulation of Ras protein signal transduction [GO:0046580] Definition: An intracellular signaling cassette in which a small monomeric GTPase of the Ras subfamily relays a signal. Sources: GOC:bf Relationships: is a type of small GTPase-mediated signal transduction [GO:0007264]